{
  "gene": "UniProtKB:Q13519",
  "term_label": "dendrite",
  "gene_symbol": "PNOC",
  "gene_name": "Prepronociceptin",
  "term_id": "GO:0030425"
}